{
  "term_id": "GO:0005886",
  "gene_symbol": "CHRNA5",
  "gene": "UniProtKB:P30532",
  "gene_name": "Neuronal acetylcholine receptor subunit alpha-5",
  "term_label": "plasma membrane"
}